diaminopimelate transport [GO:0015830] (biological process) Definition: The directed movement of diaminopimelate, the anion of 2,6-diaminoheptanedioic acid, into, out of or within a cell, or between cells, by means of some agent such as a transporter or pore. Sources: GOC:go_curators, ISBN:0198506732 Relationships: is a type of GO:0046942; is a type of nitrogen compound transport [GO:0071705]; is a type of fatty acid derivative transport [GO:1901571]